{
  "gene": "UniProtKB:Q5RKV6",
  "term_label": "nuclear exosome (RNase complex)",
  "gene_symbol": "EXOSC6",
  "term_id": "GO:0000176",
  "gene_name": "Exosome complex component MTR3"
}